{
  "term_id": "GO:0098553",
  "term_label": "lumenal side of endoplasmic reticulum membrane",
  "gene_name": "Signal peptide peptidase-like 3",
  "gene": "UniProtKB:Q8TCT6",
  "gene_symbol": "SPPL3"
}